{
  "gene_symbol": "MUC2",
  "gene": "UniProtKB:Q02817",
  "gene_name": "Mucin-2",
  "term_label": "Unknown biological process",
  "term_id": "UNKNOWN:0002"
}